{
  "gene_symbol": "UHMK1",
  "gene": "UniProtKB:Q8TAS1",
  "gene_name": "Serine_threonine-protein kinase Kist",
  "term_label": "neuronal ribonucleoprotein granule",
  "term_id": "GO:0071598"
}